L-rhamnonate dehydratase activity [GO:0050032] (molecular function) Sources: EC:4.2.1.90, RHEA:23080 Relationships: is a type of hydro-lyase activity [GO:0016836] Also known as: L-rhamnonate hydro-lyase (2-dehydro-3-deoxy-L-rhamnonate-forming), L-rhamnonate hydro-lyase activity Definition: Catalysis of the reaction: L-rhamnonate = 2-dehydro-3-deoxy-L-rhamnonate + H2O.